cardiac atrium morphogenesis [GO:0003209] (biological process) Relationships: is a type of cardiac chamber morphogenesis [GO:0003206]; is part of cardiac atrium development [GO:0003230] Subtypes: GO:0003212, cardiac right atrium morphogenesis [GO:0003213] Definition: The process in which the cardiac atrium is generated and organized. A cardiac atrium receives blood from a vein and pumps it to a cardiac ventricle. Sources: GOC:mtg_heart